{
  "term_label": "inhibitory synapse",
  "term_id": "GO:0060077",
  "gene_symbol": "LHFPL4",
  "gene": "UniProtKB:Q7Z7J7",
  "gene_name": "LHFPL tetraspan subfamily member 4 protein"
}